{
  "gene_symbol": "RIMKLA",
  "gene_name": "N-acetylaspartylglutamate synthase A",
  "term_label": "Unknown biological process",
  "term_id": "UNKNOWN:0002",
  "gene": "UniProtKB:Q8IXN7"
}